tRNA wobble base cytosine methylation [GO:0002127] (biological process) Sources: GOC:hjd, ISBN:155581073X Definition: The process in which the base of cytosine at position 34 in the anticodon of a tRNA is post-transcriptionally methylated at the C5 position. Relationships: is a type of GO:0002101; is a type of tRNA C5-cytosine methylation [GO:0002946] Also known as: wobble position m5C biosynthesis